{
  "gene_symbol": "RARRES1",
  "term_id": "UNKNOWN:0002",
  "gene": "UniProtKB:P49788",
  "term_label": "Unknown biological process",
  "gene_name": "Retinoic acid receptor responder protein 1"
}